{
  "gene_name": "Microsomal glutathione S-transferase 2",
  "term_id": "GO:0005783",
  "term_label": "endoplasmic reticulum",
  "gene_symbol": "MGST2",
  "gene": "UniProtKB:Q99735"
}